{
  "gene": "UniProtKB:P18847",
  "term_label": "DNA-binding transcription factor activity, RNA polymerase II-specific",
  "term_id": "GO:0000981",
  "gene_name": "Cyclic AMP-dependent transcription factor ATF-3",
  "gene_symbol": "ATF3"
}